alkylmercury lyase activity [GO:0018836] (molecular function) Definition: Catalysis of the reaction: an alkylmercury + H+ = an alkane + Hg2+. Also known as: alkylmercury mercuric-lyase (alkane-forming), alkylmercury mercuric-lyase activity, organomercurial lyase activity, organomercury lyase activity Relationships: is a type of GO:0016829 Sources: RHEA:18777